{
  "gene_name": "DNA polymerase alpha catalytic subunit",
  "gene_symbol": "POLA1",
  "term_id": "GO:0003682",
  "gene": "UniProtKB:P09884",
  "term_label": "chromatin binding"
}